{
  "gene_symbol": "CACNG1",
  "gene": "UniProtKB:Q06432",
  "term_id": "GO:1990454",
  "term_label": "L-type voltage-gated calcium channel complex",
  "gene_name": "Voltage-dependent calcium channel gamma-1 subunit"
}